{
  "gene_name": "Neuronal acetylcholine receptor subunit alpha-6",
  "term_id": "GO:0035094",
  "gene": "UniProtKB:Q15825",
  "term_label": "response to nicotine",
  "gene_symbol": "CHRNA6"
}